{
  "term_label": "regulation of transcription by RNA polymerase II",
  "term_id": "GO:0006357",
  "gene_name": "Vascular endothelial zinc finger 1",
  "gene_symbol": "VEZF1",
  "gene": "UniProtKB:Q14119"
}